renal tubule development [GO:0061326] (biological process) Sources: GOC:dph, GOC:mtg_kidney_jan10 Relationships: is a type of tube development [GO:0035295]; is a type of epithelium development [GO:0060429]; is part of renal system development [GO:0072001] Subtypes: GO:0072002, nephron tubule development [GO:0072080] Definition: The progression of the renal tubule over time from its formation to the mature form. A renal tubule is a tube that filters, re-absorbs and secretes substances to rid an organism of waste and to play a role in fluid homeostasis.